{
  "gene_symbol": "OR51D1",
  "gene_name": "Olfactory receptor 51D1",
  "term_id": "GO:0004984",
  "gene": "UniProtKB:Q8NGF3",
  "term_label": "olfactory receptor activity"
}